{
  "term_id": "UNKNOWN:0002",
  "gene_name": "Protein CASC3",
  "term_label": "Unknown biological process",
  "gene_symbol": "CASC3",
  "gene": "UniProtKB:O15234"
}